{
  "gene_name": "C-C motif chemokine 22",
  "term_id": "GO:0008009",
  "gene": "UniProtKB:O00626",
  "term_label": "chemokine activity",
  "gene_symbol": "CCL22"
}